{
  "gene_symbol": "SEMA4D",
  "term_id": "GO:0045499",
  "gene_name": "Semaphorin-4D",
  "term_label": "chemorepellent activity",
  "gene": "UniProtKB:Q92854"
}